{
  "gene_symbol": "TP53INP1",
  "gene": "UniProtKB:Q96A56",
  "term_id": "UNKNOWN:0001",
  "term_label": "Unknown molecular function",
  "gene_name": "Tumor protein p53-inducible nuclear protein 1"
}